positive regulation of pheromone response MAPK cascade [GO:0062038] (biological process) Relationships: is a type of positive regulation of MAPK cascade [GO:0043410]; is a type of regulation of pheromone response MAPK cascade [GO:0180039]; positively regulates pheromone response MAPK cascade [GO:0071507] References: PMID:9315645 Definition: Any process that activates or increases the frequency, rate or extent of a pheromone response MAPK cascade.